R1/R6 development [GO:0048053] (biological process) Relationships: is a type of compound eye photoreceptor development [GO:0042051]; is part of R1/R6 cell differentiation [GO:0048052] Sources: GOC:jid Definition: The process whose specific outcome is the progression of the R1 and R6 pair of photoreceptors in the eye over time, from their formation to the mature structures. R1 and R6 are paired photoreceptors that contribute to the outer rhabdomeres. An example of this process is found in Drosophila melanogaster.